positive regulation of catabolic process [GO:0009896] (biological process) Sources: GOC:go_curators Also known as: positive regulation of breakdown, positive regulation of catabolism, positive regulation of degradation, up regulation of catabolic process, up-regulation of catabolic process, upregulation of catabolic process, activation of catabolic process, stimulation of catabolic process Relationships: is a type of positive regulation of metabolic process [GO:0009893]; is a type of regulation of catabolic process [GO:0009894]; positively regulates GO:0009056 Subtypes: positive regulation of mitochondrial RNA catabolic process [GO:0000962], positive regulation of autophagy [GO:0010508], GO:0030813, positive regulation of amine catabolic process [GO:0033243], positive regulation of penicillin catabolic process [GO:0033249], GO:0034253, positive regulation of protein catabolic process [GO:0045732], positive regulation of acetate catabolic process [GO:0045754], positive regulation of glycogen catabolic process [GO:0045819], RNA destabilization [GO:0050779], GO:0050996, positive regulation of mRNA catabolic process [GO:0061014], GO:0120158, GO:0160159, positive regulation of nicotine catabolic process [GO:0160160], positive regulation of anthocyanin catabolic process [GO:1900002], positive regulation of cellobiose catabolic process [GO:1900284], positive regulation of coenzyme F420-dependent bicyclic nitroimidazole catabolic process [GO:1900290], positive regulation of alcohol catabolic process [GO:1900421], positive regulation of xylose catabolic process to ethanol [GO:1900517], positive regulation of trehalose catabolic process [GO:1901319], positive regulation of tetrapyrrole catabolic process [GO:1901406], positive regulation of toluene catabolic process [GO:1901436], positive regulation of ferulate catabolic process [GO:1901468], positive regulation of syringal lignin catabolic process [GO:1901471], positive regulation of gamma-aminobutyric acid catabolic process [GO:1901717], GO:1902372, GO:1903268, positive regulation of hydrogen peroxide catabolic process [GO:1903285], positive regulation of DNA catabolic process [GO:1903626], positive regulation of glucose catabolic process to lactate via pyruvate [GO:1904025], positive regulation of ubiquitin-dependent protein catabolic process [GO:2000060], positive regulation of miRNA catabolic process [GO:2000627], positive regulation of receptor catabolic process [GO:2000646], positive regulation of starch catabolic process [GO:2000883], GO:2000914, positive regulation of cellodextrin catabolic process [GO:2000929], positive regulation of cellotriose catabolic process [GO:2000938], positive regulation of cyclodextrin catabolic process [GO:2000959], positive regulation of cellooligosaccharide catabolic process [GO:2000965], positive regulation of cell wall polysaccharide catabolic process [GO:2000968], positive regulation of hemicellulose catabolic process [GO:2000990], positive regulation of galactomannan catabolic process [GO:2000993], GO:2000999, positive regulation of pectin catabolic process [GO:2001005], positive regulation of L-proline catabolic process to L-glutamate [GO:2001158], positive regulation of glycolytic fermentation to ethanol [GO:2001172] Definition: Any process that activates or increases the frequency, rate or extent of the chemical reactions and pathways resulting in the breakdown of substances.